{
  "gene_name": "Polyamine-transporting ATPase 13A2",
  "term_label": "polyamine transmembrane transporter activity",
  "gene": "UniProtKB:Q9NQ11",
  "term_id": "GO:0015203",
  "gene_symbol": "ATP13A2"
}